{
  "term_label": "negative regulation of transcription by RNA polymerase II",
  "gene_symbol": "ZGPAT",
  "term_id": "GO:0000122",
  "gene": "UniProtKB:Q8N5A5",
  "gene_name": "Zinc finger CCCH-type with G patch domain-containing protein"
}